{
  "term_label": "basolateral plasma membrane",
  "gene_name": "Disks large homolog 2",
  "gene": "UniProtKB:Q15700",
  "term_id": "GO:0016323",
  "gene_symbol": "DLG2"
}